{
  "gene_name": "Mitochondrial tRNA-specific 2-thiouridylase 1",
  "term_id": "GO:0005739",
  "gene": "UniProtKB:O75648",
  "term_label": "mitochondrion",
  "gene_symbol": "TRMU"
}